{
  "gene_symbol": "TAF3",
  "gene": "UniProtKB:Q5VWG9",
  "gene_name": "Transcription initiation factor TFIID subunit 3",
  "term_id": "GO:0045944",
  "term_label": "positive regulation of transcription by RNA polymerase II"
}